ceramide transport [GO:0035627] (biological process) Definition: The directed movement of ceramides into, out of or within a cell, or between cells, by means of some agent such as a transporter or pore. Ceramides are a class of lipid composed of sphingosine linked to a fatty acid. Sources: GOC:bf, GOC:sart Relationships: is a type of GO:0006869; is a type of GO:0042886 Subtypes: ER to Golgi ceramide transport [GO:0035621], GO:0099040, ceramide 1-phosphate transport [GO:1902389], GO:1905572